{
  "term_label": "intracellular signal transduction",
  "gene": "UniProtKB:Q12851",
  "gene_symbol": "MAP4K2",
  "term_id": "GO:0035556",
  "gene_name": "Mitogen-activated protein kinase kinase kinase kinase 2"
}